cellular response to staurosporine [GO:0072734] (biological process) Relationships: is a type of cellular response to alkaloid [GO:0071312]; is a type of GO:0072733 Sources: GOC:mah Definition: Any process that results in a change in state or activity of a cell (in terms of movement, secretion, enzyme production, gene expression, etc.) as a result of a staurosporine stimulus.